{
  "term_label": "Unknown molecular function",
  "gene_symbol": "NDUFB7",
  "gene_name": "NADH dehydrogenase [ubiquinone] 1 beta subcomplex subunit 7",
  "gene": "UniProtKB:P17568",
  "term_id": "UNKNOWN:0001"
}